{
  "gene_name": "Peroxisomal sarcosine oxidase",
  "gene_symbol": "PIPOX",
  "gene": "UniProtKB:Q9P0Z9",
  "term_label": "sarcosine oxidase activity",
  "term_id": "GO:0008115"
}